emericellin catabolic process [GO:1900765] (biological process) Relationships: is a type of phenol-containing compound catabolic process [GO:0019336]; is a type of ketone catabolic process [GO:0042182]; is a type of secondary metabolite catabolic process [GO:0090487]; is a type of ether catabolic process [GO:1901502] Sources: GOC:TermGenie, GOC:di Definition: The chemical reactions and pathways resulting in the breakdown of emericellin. Also known as: emericellin breakdown, emericellin catabolism, emericellin degradation, Variecoxanthone B breakdown, Variecoxanthone B catabolic process, Variecoxanthone B catabolism, Variecoxanthone B degradation